{
  "gene_symbol": "ERAP1",
  "term_id": "GO:0070006",
  "term_label": "metalloaminopeptidase activity",
  "gene": "UniProtKB:Q9NZ08",
  "gene_name": "Endoplasmic reticulum aminopeptidase 1"
}